{
  "gene_symbol": "CYP11B1",
  "gene_name": "Cytochrome P450 11B1, mitochondrial",
  "gene": "UniProtKB:P15538",
  "term_id": "GO:0006704",
  "term_label": "glucocorticoid biosynthetic process"
}